{
  "term_label": "xylosyl alpha-1,3-xylosyltransferase activity",
  "gene": "UniProtKB:Q8NBI6",
  "term_id": "GO:0140560",
  "gene_symbol": "XXYLT1",
  "gene_name": "Xyloside xylosyltransferase 1"
}